{
  "term_label": "Unknown cellular component",
  "gene": "UniProtKB:Q96BN6",
  "gene_name": "Primary cilium assembly protein FAM149B1",
  "gene_symbol": "FAM149B1",
  "term_id": "UNKNOWN:0003"
}